glutamate-ethylamine ligase activity [GO:0047942] (molecular function) Sources: EC:6.3.1.6, RHEA:20525 Definition: Catalysis of the reaction: L-glutamate + ATP + ethylamine = N(5)-ethyl-L-glutamine + ADP + 2 H+ + phosphate. Relationships: is a type of acid-ammonia (or amide) ligase activity [GO:0016880] Also known as: L-glutamate:ethylamine ligase (ADP-forming), N(5)-ethyl-L-glutamine synthetase activity, N5-ethyl-L-glutamine synthetase activity, N5-ethylglutamine synthetase activity, theanine synthetase activity